{
  "gene": "UniProtKB:P09693",
  "gene_symbol": "CD3G",
  "gene_name": "T-cell surface glycoprotein CD3 gamma chain",
  "term_id": "GO:0004888",
  "term_label": "transmembrane signaling receptor activity"
}